{
  "term_id": "UNKNOWN:0003",
  "term_label": "Unknown cellular component",
  "gene_symbol": "GCNT4",
  "gene_name": "Beta-1,3-galactosyl-O-glycosyl-glycoprotein beta-1,6-N-acetylglucosaminyltransferase 4",
  "gene": "UniProtKB:Q9P109"
}